negative regulation of tolerance induction [GO:0002644] (biological process) Definition: Any process that stops, prevents, or reduces the frequency, rate, or extent of tolerance induction. Relationships: is a type of regulation of tolerance induction [GO:0002643]; is a type of negative regulation of immune system process [GO:0002683]; is a type of negative regulation of developmental process [GO:0051093]; is a type of GO:0051241; RO_0002212 tolerance induction [GO:0002507] Also known as: down regulation of tolerance induction, down-regulation of tolerance induction, downregulation of tolerance induction, inhibition of tolerance induction Sources: GOC:add Subtypes: negative regulation of central tolerance induction [GO:0002647], negative regulation of tolerance induction to self antigen [GO:0002650], negative regulation of tolerance induction dependent upon immune response [GO:0002653], negative regulation of B cell tolerance induction [GO:0002662], negative regulation of T cell tolerance induction [GO:0002665], negative regulation of natural killer cell tolerance induction [GO:0002872], negative regulation of lymphocyte anergy [GO:0002912]